glutamate receptor signaling pathway [GO:0007215] (biological process) Also known as: glutamate signaling pathway, glutamate signalling pathway Subtypes: GO:0007216, ionotropic glutamate receptor signaling pathway [GO:0035235] Definition: The series of molecular signals initiated by the binding of glutamate to its receptor on the surface of a target cell, and ending with the regulation of a downstream cellular process, e.g. transcription. Relationships: is a type of cell surface receptor signaling pathway [GO:0007166]; has part glutamate receptor activity [GO:0008066] Regulation: regulated by regulation of glutamate receptor signaling pathway [GO:1900449]; RO_0002212 by negative regulation of glutamate receptor signaling pathway [GO:1900450]; positively regulated by positive regulation of glutamate receptor signaling pathway [GO:1900451] References: PMID:9131252 Sources: GOC:mah, GOC:signaling